{
  "term_label": "synaptic vesicle budding from endosome",
  "term_id": "GO:0016182",
  "gene_name": "AP-3 complex subunit delta-1",
  "gene_symbol": "AP3D1",
  "gene": "UniProtKB:O14617"
}